{
  "term_label": "T cell extravasation",
  "term_id": "GO:0072683",
  "gene_name": "Glycoprotein Xg",
  "gene": "UniProtKB:P55808",
  "gene_symbol": "XG"
}